{
  "gene_symbol": "GRAMD1B",
  "gene": "UniProtKB:Q3KR37",
  "term_label": "cholesterol binding",
  "term_id": "GO:0015485",
  "gene_name": "Protein Aster-B"
}